chitin deacetylase activity [GO:0004099] (molecular function) Sources: EC:3.5.1.41 Definition: Catalysis of the reaction: chitin + H2O = chitosan + acetate. Also known as: chitin amidohydrolase activity Relationships: is a type of GO:0016811; is a type of deacetylase activity [GO:0019213]